{
  "gene_symbol": "MFSD14A",
  "gene": "UniProtKB:Q96MC6",
  "term_id": "UNKNOWN:0001",
  "gene_name": "Hippocampus abundant transcript 1 protein",
  "term_label": "Unknown molecular function"
}